{
  "gene": "UniProtKB:Q9UKY7",
  "term_id": "UNKNOWN:0002",
  "gene_symbol": "CDV3",
  "gene_name": "Protein CDV3 homolog",
  "term_label": "Unknown biological process"
}